DCT cell differentiation [GO:0072069] (biological process) Relationships: is a type of cell differentiation involved in kidney development [GO:0061005]; is part of distal convoluted tubule development [GO:0072025] Definition: The process in which relatively unspecialized cells acquire specialized structural and/or functional features that characterize the distal convoluted tubule cells of the kidney as it progresses from its formation to the mature state. Also known as: distal convoluted tubule cell differentiation Sources: GOC:mtg_kidney_jan10 Subtypes: GO:0072240